{
  "term_label": "chromatin binding",
  "gene_symbol": "ASXL3",
  "gene": "UniProtKB:Q9C0F0",
  "term_id": "GO:0003682",
  "gene_name": "Putative Polycomb group protein ASXL3"
}